protein insertion into ER membrane by internal uncleaved signal-anchor sequence [GO:0045051] (biological process) Definition: A process of protein insertion into the endoplasmic reticulum (ER) membrane in which signal anchor sequences function as both ER signal sequences and membrane anchor sequences. Sources: ISBN:0716731363 Also known as: internal uncleaved signal-anchor sequence mediated protein insertion into ER membrane, protein insertion into ER membrane, internal uncleaved signal-anchor sequence mediated, protein insertion into endoplasmic reticulum membrane by internal uncleaved signal-anchor sequence, protein-ER insertion by internal uncleaved signal-anchor sequence, protein-endoplasmic reticulum insertion by internal uncleaved signal-anchor sequence Relationships: is a type of GO:0045048